kojic acid biosynthetic process [GO:2001317] (biological process) Definition: The chemical reactions and pathways resulting in the formation of kojic acid. Sources: GOC:di Regulation: RO_0002211 by regulation of kojic acid biosynthetic process [GO:1900394]; negatively regulated by negative regulation of kojic acid biosynthetic process [GO:1900395]; positively regulated by GO:1900396 Relationships: is a type of primary alcohol biosynthetic process [GO:0034309]; is a type of ketone biosynthetic process [GO:0042181]; is_a olefinic compound biosynthetic process [GO:0120255] Also known as: 5-hydroxy-2-(hydroxymethyl)-4H-pyran-4-one anabolism, 5-hydroxy-2-(hydroxymethyl)-4H-pyran-4-one biosynthesis, 5-hydroxy-2-(hydroxymethyl)-4H-pyran-4-one biosynthetic process, 5-hydroxy-2-(hydroxymethyl)-4H-pyran-4-one formation, 5-hydroxy-2-(hydroxymethyl)-4H-pyran-4-one synthesis, kojic acid anabolism, kojic acid biosynthesis, kojic acid formation, kojic acid synthesis, C6H6O4 anabolism, C6H6O4 biosynthesis, C6H6O4 biosynthetic process, C6H6O4 formation, C6H6O4 synthesis